{
  "term_label": "negative regulation of inflammatory response",
  "gene_name": "Peroxisome proliferator-activated receptor alpha",
  "term_id": "GO:0050728",
  "gene": "UniProtKB:Q07869",
  "gene_symbol": "PPARA"
}